{
  "term_label": "Unknown cellular component",
  "gene": "UniProtKB:Q8NDY4",
  "gene_name": "Myelodysplastic syndrome 2 translocation-associated protein",
  "gene_symbol": "MDS2",
  "term_id": "UNKNOWN:0003"
}